interphotoreceptor matrix [GO:0033165] (cellular component) Definition: A specialized extracellularc matrix that surrounds the photoreceptors of the retina and lies between them and the apical surface of the retinal pigment epithelium. The IPM has been implicated in several important activities required for photoreceptor function and maintenance. References: PMID:1862095, PMID:2194288 Relationships: is_a specialized extracellular matrix [GO:0140047]